response to light intensity [GO:0009642] (biological process) Subtypes: photosynthetic acclimation [GO:0009643], response to high light intensity [GO:0009644], response to low light intensity stimulus [GO:0009645], response to absence of light [GO:0009646], light adaption [GO:0036367], response to very low light intensity stimulus [GO:0055122], GO:0071484, GO:0120302 Sources: GOC:go_curators Relationships: is_a response to light stimulus [GO:0009416] Definition: Any process that results in a change in state or activity of a cell or an organism (in terms of movement, secretion, enzyme production, gene expression, etc.) as a result of a light intensity stimulus.